regulation of skeletal muscle tissue regeneration [GO:0043416] (biological process) Subtypes: regulation of satellite cell activation involved in skeletal muscle regeneration [GO:0014717], positive regulation of skeletal muscle tissue regeneration [GO:0043415], negative regulation of skeletal muscle tissue regeneration [GO:0043417] Sources: GOC:jl Definition: Any process that modulates the frequency, rate or extent of skeletal muscle. Relationships: is a type of regulation of response to external stimulus [GO:0032101]; is a type of regulation of developmental growth [GO:0048638]; is a type of regulation of multicellular organismal development [GO:2000026]; regulates skeletal muscle tissue regeneration [GO:0043403]